{
  "gene_name": "Patatin-like phospholipase domain-containing protein 5",
  "term_label": "lipid homeostasis",
  "gene": "UniProtKB:Q7Z6Z6",
  "term_id": "GO:0055088",
  "gene_symbol": "PNPLA5"
}